{
  "gene_symbol": "COPZ2",
  "term_label": "intracellular protein transport",
  "gene": "UniProtKB:Q9P299",
  "gene_name": "Coatomer subunit zeta-2",
  "term_id": "GO:0006886"
}